{
  "term_label": "SNARE complex",
  "term_id": "GO:0031201",
  "gene": "UniProtKB:P56962",
  "gene_name": "Syntaxin-17",
  "gene_symbol": "STX17"
}